{
  "gene_symbol": "LRRC42",
  "gene": "UniProtKB:Q9Y546",
  "term_id": "UNKNOWN:0001",
  "term_label": "Unknown molecular function",
  "gene_name": "Leucine-rich repeat-containing protein 42"
}